{
  "gene_name": "Microfibrillar-associated protein 3-like",
  "term_id": "UNKNOWN:0001",
  "term_label": "Unknown molecular function",
  "gene": "UniProtKB:O75121",
  "gene_symbol": "MFAP3L"
}